negative regulation of CD8-positive, alpha-beta T cell proliferation [GO:2000565] (biological process) Definition: Any process that stops, prevents or reduces the frequency, rate or extent of CD8-positive, alpha-beta T cell proliferation. Sources: GOC:obol Relationships: is a type of negative regulation of alpha-beta T cell proliferation [GO:0046642]; is a type of regulation of CD8-positive, alpha-beta T cell proliferation [GO:2000564]; is a type of GO:2001186; negatively regulates CD8-positive, alpha-beta T cell proliferation [GO:0035740]